{
  "term_label": "nucleus",
  "gene_symbol": "ZNF420",
  "term_id": "GO:0005634",
  "gene": "UniProtKB:Q8TAQ5",
  "gene_name": "Zinc finger protein 420"
}